{
  "term_label": "membrane depolarization",
  "gene": "UniProtKB:P30532",
  "gene_symbol": "CHRNA5",
  "term_id": "GO:0051899",
  "gene_name": "Neuronal acetylcholine receptor subunit alpha-5"
}